{
  "term_id": "GO:0007165",
  "gene_symbol": "MOB2",
  "gene": "UniProtKB:Q70IA6",
  "term_label": "signal transduction",
  "gene_name": "MOB kinase activator 2"
}